{
  "gene_symbol": "RASA1",
  "gene_name": "Ras GTPase-activating protein 1",
  "gene": "UniProtKB:P20936",
  "term_id": "GO:1902531",
  "term_label": "regulation of intracellular signal transduction"
}